{
  "term_id": "GO:0007368",
  "term_label": "determination of left/right symmetry",
  "gene_name": "Nephrocystin-3",
  "gene": "UniProtKB:Q7Z494",
  "gene_symbol": "NPHP3"
}